{
  "gene": "UniProtKB:P04150",
  "gene_symbol": "NR3C1",
  "term_label": "chromatin",
  "term_id": "GO:0000785",
  "gene_name": "Glucocorticoid receptor"
}